{
  "term_label": "Unknown biological process",
  "gene_name": "Cancer-related nucleoside-triphosphatase",
  "term_id": "UNKNOWN:0002",
  "gene_symbol": "NTPCR",
  "gene": "UniProtKB:Q9BSD7"
}